{
  "gene": "UniProtKB:Q15669",
  "gene_name": "Rho-related GTP-binding protein RhoH",
  "term_label": "GTPase activity",
  "gene_symbol": "RHOH",
  "term_id": "GO:0003924"
}